{
  "gene_symbol": "PALB2",
  "term_label": "DNA binding",
  "term_id": "GO:0003677",
  "gene": "UniProtKB:Q86YC2",
  "gene_name": "Partner and localizer of BRCA2"
}